{
  "gene": "UniProtKB:Q8NA29",
  "term_id": "GO:1990379",
  "term_label": "lipid transport across blood-brain barrier",
  "gene_symbol": "MFSD2A",
  "gene_name": "Sodium-dependent lysophosphatidylcholine symporter 1"
}